pyrimidine ribonucleotide interconversion [GO:0015954] (biological process) Sources: GOC:mah, ISBN:0306444747, ISBN:0471394831 Relationships: is a type of pyrimidine ribonucleotide metabolic process [GO:0009218]; is a type of pyrimidine nucleotide interconversion [GO:0015953] Definition: The chemical reactions and pathways by which a pyrimidine ribonucleotide is synthesized from another pyrimidine ribonucleotide.